{
  "term_label": "guanyl-nucleotide exchange factor activity",
  "gene_name": "MAP kinase-activating death domain protein",
  "gene_symbol": "MADD",
  "gene": "UniProtKB:Q8WXG6",
  "term_id": "GO:0005085"
}